{
  "term_label": "Golgi apparatus",
  "gene_symbol": "B4GALT1",
  "term_id": "GO:0005794",
  "gene_name": "Beta-1,4-galactosyltransferase 1",
  "gene": "UniProtKB:P15291"
}